{
  "term_label": "aldehyde catabolic process",
  "gene_symbol": "ALDH2",
  "gene_name": "Aldehyde dehydrogenase, mitochondrial",
  "term_id": "GO:0046185",
  "gene": "UniProtKB:P05091"
}